{
  "gene_symbol": "SYT6",
  "gene": "UniProtKB:Q5T7P8",
  "term_label": "regulation of calcium ion-dependent exocytosis",
  "term_id": "GO:0017158",
  "gene_name": "Synaptotagmin-6"
}